{
  "gene_name": "Myeloid cell nuclear differentiation antigen",
  "gene_symbol": "MNDA",
  "term_id": "GO:0005654",
  "gene": "UniProtKB:P41218",
  "term_label": "nucleoplasm"
}